{
  "gene_symbol": "UNC45A",
  "gene_name": "Protein unc-45 homolog A",
  "term_id": "GO:0051879",
  "gene": "UniProtKB:Q9H3U1",
  "term_label": "Hsp90 protein binding"
}